histone methyltransferase activity [GO:0042054] (molecular function) Sources: GOC:curators Also known as: histone N-methyltransferase activity, histone methylase activity Subtypes: GO:0140188, histone H3 methyltransferase activity [GO:0140938], histone H4 methyltransferase activity [GO:0140939], histone H2A methyltransferase activity [GO:0140940] Definition: Catalysis of the reaction: S-adenosyl-L-methionine + histone = S-adenosyl-L-homocysteine + methyl-histone. Histone methylation generally occurs on either an arginine or a lysine residue. Relationships: is a type of protein methyltransferase activity [GO:0008276]; is a type of GO:0140993